{
  "gene_name": "HLA class I histocompatibility antigen, alpha chain G",
  "term_label": "extracellular space",
  "gene": "UniProtKB:P17693",
  "gene_symbol": "HLA-G",
  "term_id": "GO:0005615"
}